{
  "gene_name": "Probable ATP-dependent RNA helicase DDX4",
  "term_id": "GO:0007276",
  "term_label": "gamete generation",
  "gene_symbol": "DDX4",
  "gene": "UniProtKB:Q9NQI0"
}